{
  "gene": "UniProtKB:O14978",
  "gene_name": "Zinc finger protein 263",
  "gene_symbol": "ZNF263",
  "term_id": "GO:0000978",
  "term_label": "RNA polymerase II cis-regulatory region sequence-specific DNA binding"
}